glycerol-2-phosphate transmembrane transport [GO:0070811] (biological process) Also known as: glycerol-2-phosphate transport Sources: GOC:mah Definition: The process in which glycerol-2-phosphate is transported across a membrane. Glycerol-2-phosphate is a phosphoric monoester of glycerol. Relationships: is a type of organic anion transport [GO:0015711]; is a type of organophosphate ester transport [GO:0015748]; is a type of transmembrane transport [GO:0055085]; is a type of GO:1901264